posterior lateral line neuromast hair cell development [GO:0035677] (biological process) Definition: The process whose specific outcome is the progression of a posterior lateral line neuromast hair cell over time, from its formation to the mature structure. A neuromast hair cell is a hair cell that acts as a sensory receptor of the neuromast; it is morphologically polarized as a result of the relative position of the single kinocilium and the clusters of stereocilia on its apical surface. Cell development does not include the steps involved in committing a cell to a specific fate. Relationships: is a type of GO:0035675; is part of posterior lateral line neuromast hair cell differentiation [GO:0048923] Sources: ISBN:0125296509